cone cell pedicle [GO:0044316] (cellular component) Definition: A specialized axon terminus which is produced by retinal cone cells. Pedicles are large, conical, flat end-feet (8-10 micrometers diameter) of the retinal cone axon that lie more or less side by side on the same plane at the outer edge of the outer plexiform layer (OPL). References: PMID:10939333 Also known as: cone pedicle Relationships: is a type of axon terminus [GO:0043679]